{
  "term_id": "UNKNOWN:0001",
  "gene_name": "Ankyrin repeat and SOCS box protein 18",
  "gene": "UniProtKB:Q6ZVZ8",
  "gene_symbol": "ASB18",
  "term_label": "Unknown molecular function"
}